phosphoribosylaminoimidazolesuccinocarboxamide synthase activity [GO:0004639] (molecular function) Definition: Catalysis of the reaction: 5-amino-1-(5-phospho-D-ribosyl)imidazole-4-carboxylate + L-aspartate + ATP = (2S)-2-[5-amino-1-(5-phospho-beta-D-ribosyl)imidazole-4-carboxamido]succinate + ADP + 2 H+ + phosphate. Also known as: 4-((N-succinylamino)carbonyl)-5-aminoimidazole ribonucleotide synthetase activity, 4-(N-succinocarboxamide)-5-aminoimidazole synthetase activity, 4-[(N-succinylamino)carbonyl]-5-aminoimidazole ribonucleotide synthetase activity, 5-amino-1-(5-phospho-D-ribosyl)imidazole-4-carboxylate:L-aspartate ligase (ADP-forming), 5-aminoimidazole-4-N-succinocarboxamide ribonucleotide synthetase activity, PurC, SAICAR synthase activity, SAICAR synthetase activity, SAICARs activity, phosphoribosylaminoimidazole-succinocarboxamide synthase activity, phosphoribosylaminoimidazole-succinocarboxamide synthetase activity, phosphoribosylaminoimidazolesuccinocarboxamide synthetase activity Relationships: is a type of acid-amino acid ligase activity [GO:0016881] Sources: EC:6.3.2.6, RHEA:22628